{
  "gene_name": "Synapse differentiation-inducing gene protein 1",
  "term_id": "GO:0060076",
  "gene_symbol": "SYNDIG1",
  "gene": "UniProtKB:Q9H7V2",
  "term_label": "excitatory synapse"
}